{
  "term_label": "DNA-binding transcription repressor activity, RNA polymerase II-specific",
  "term_id": "GO:0001227",
  "gene_symbol": "FOXP2",
  "gene": "UniProtKB:O15409",
  "gene_name": "Forkhead box protein P2"
}